{
  "gene_name": "RRP12-like protein",
  "term_id": "UNKNOWN:0002",
  "term_label": "Unknown biological process",
  "gene": "UniProtKB:Q5JTH9",
  "gene_symbol": "RRP12"
}